response to dehydroepiandrosterone [GO:1903494] (BP) References: PMID:3585228 Sources: GOC:TermGenie, GOC:mr, GO_REF:0000071 Relationships: is a type of response to lipid [GO:0033993]; is a type of GO:0097305; is a type of GO:1901654 Subtypes: cellular response to dehydroepiandrosterone [GO:1903495] Definition: Any process that results in a change in state or activity of a cell or an organism (in terms of movement, secretion, enzyme production, gene expression, etc.) as a result of a dehydroepiandrosterone stimulus.